{
  "gene": "UniProtKB:P49005",
  "term_label": "Unknown molecular function",
  "gene_symbol": "POLD2",
  "term_id": "UNKNOWN:0001",
  "gene_name": "DNA polymerase delta subunit 2"
}